{
  "gene": "UniProtKB:O15391",
  "term_id": "GO:0000981",
  "gene_name": "Transcription factor YY2",
  "gene_symbol": "YY2",
  "term_label": "DNA-binding transcription factor activity, RNA polymerase II-specific"
}